terpenoid biosynthetic process [GO:0016114] (biological process) Subtypes: monoterpenoid biosynthetic process [GO:0016099], diterpenoid biosynthetic process [GO:0016102], GO:0016104, sesquiterpenoid biosynthetic process [GO:0016106], tetraterpenoid biosynthetic process [GO:0016109], GO:0016112, GDP-alpha-D-mannosylchitobiosyldiphosphodolichol biosynthetic process [GO:0019347], geranyl diphosphate biosynthetic process [GO:0033384], geranylgeranyl diphosphate biosynthetic process [GO:0033386], phytyl diphosphate biosynthetic process [GO:0033521], 4-amino-4-deoxy-alpha-L-arabinopyranosyl undecaprenyl phosphate biosynthetic process [GO:0036108], farnesyl diphosphate biosynthetic process [GO:0045337], trisporic acid biosynthetic process [GO:0046842], terpenoid biosynthetic process, mevalonate-independent [GO:0051483], terpenoid biosynthetic process, mevalonate-dependent [GO:0051485], novofumigatonin biosynthetic process [GO:0140782], GO:0140874, GO:0180047 Relationships: is a type of terpenoid metabolic process [GO:0006721]; is a type of isoprenoid biosynthetic process [GO:0008299] Also known as: terpenoid anabolism, terpenoid biosynthesis, terpenoid formation, terpenoid synthesis Definition: The chemical reactions and pathways resulting in the formation of terpenoids, any member of a class of compounds characterized by an isoprenoid chemical structure. Sources: GOC:ai